{
  "term_id": "UNKNOWN:0003",
  "term_label": "Unknown cellular component",
  "gene_name": "Inter-alpha-trypsin inhibitor heavy chain H3",
  "gene_symbol": "ITIH3",
  "gene": "UniProtKB:Q06033"
}